{
  "gene_symbol": "CPN1",
  "term_id": "GO:0005615",
  "term_label": "extracellular space",
  "gene_name": "Carboxypeptidase N catalytic chain",
  "gene": "UniProtKB:P15169"
}